thiamine-diphosphate kinase activity [GO:0050331] (molecular function) Also known as: thiamin diphosphate kinase activity, thiamin-diphosphate kinase activity, ATP:thiamin-diphosphate phosphotransferase activity, ATP:thiamine-diphosphate phosphotransferase activity, TDP kinase activity, protein bound thiamin diphosphate:ATP phosphoryltransferase activity, thiamin diphosphate phosphotransferase activity, thiamin pyrophosphate kinase activity, thiamine diphosphate kinase activity Sources: EC:2.7.4.15, MetaCyc:THIAMIN-DIPHOSPHATE-KINASE-RXN Relationships: is a type of kinase activity [GO:0016301]; is a type of GO:0016776 Definition: Catalysis of the reaction: ATP + thiamin diphosphate = ADP + thiamin triphosphate.